{
  "term_label": "regulation of neurogenesis",
  "gene": "UniProtKB:Q9NQ87",
  "term_id": "GO:0050767",
  "gene_name": "Hairy_enhancer-of-split related with YRPW motif-like protein",
  "gene_symbol": "HEYL"
}